host cell chloroplast part [GO:0033653] (cellular component) Subtypes: GO:0033654 Definition: Any constituent part of a chloroplast as it is found in host cells and which are a chlorophyll-containing plastid with thylakoids organized into grana and frets, or stroma thylakoids, and embedded in a stroma. The host is defined as the larger of the organisms involved in a symbiotic interaction. Note: Note that this term is in the subset of terms that should not be used for direct gene product annotation. Instead, select a child term or, if no appropriate child term exists, please request a new term. Direct annotations to this term may be amended during annotation QC. Sources: GOC:pamgo_curators Relationships: is a type of GO:0033652 Also known as: host chloroplast component